{
  "term_label": "nucleus",
  "term_id": "GO:0005634",
  "gene_name": "RE1-silencing transcription factor",
  "gene": "UniProtKB:Q13127",
  "gene_symbol": "REST"
}